{
  "term_label": "Unknown biological process",
  "gene_symbol": "C1orf220",
  "gene": "UniProtKB:Q5T0J3",
  "gene_name": "Putative uncharacterized protein C1orf220",
  "term_id": "UNKNOWN:0002"
}